{
  "gene_symbol": "ARFGAP3",
  "term_id": "UNKNOWN:0003",
  "gene_name": "ADP-ribosylation factor GTPase-activating protein 3",
  "gene": "UniProtKB:Q9NP61",
  "term_label": "Unknown cellular component"
}